{
  "gene": "UniProtKB:Q8NC51",
  "gene_name": "SERPINE1 mRNA-binding protein 1",
  "term_id": "GO:0003730",
  "gene_symbol": "SERBP1",
  "term_label": "mRNA 3'-UTR binding"
}